{
  "gene_symbol": "FOXI3",
  "term_label": "regulation of transcription by RNA polymerase II",
  "gene_name": "Forkhead box protein I3",
  "gene": "UniProtKB:A8MTJ6",
  "term_id": "GO:0006357"
}